{
  "gene_name": "Golgi-associated kinase 1B",
  "gene": "UniProtKB:Q6UWH4",
  "term_label": "Golgi apparatus",
  "gene_symbol": "GASK1B",
  "term_id": "GO:0005794"
}